{
  "gene_symbol": "PNPT1",
  "gene": "UniProtKB:Q8TCS8",
  "term_id": "GO:0000175",
  "term_label": "3'-5'-RNA exonuclease activity",
  "gene_name": "Polyribonucleotide nucleotidyltransferase 1, mitochondrial"
}